{
  "term_label": "Unknown cellular component",
  "gene": "UniProtKB:K7EJ46",
  "term_id": "UNKNOWN:0003",
  "gene_name": "Small integral membrane protein 22",
  "gene_symbol": "SMIM22"
}